1-alkyl-2-acetylglycerophosphocholine esterase activity [GO:0003847] (molecular function) Definition: Catalysis of the reaction: a 1-O-alkyl-2-acetyl-sn-glycero-3-phosphocholine + H2O = 1-O-alkyl-sn-glycero-3-phosphocholine + acetate + H+. Sources: RHEA:17777 Relationships: is a type of carboxylic ester hydrolase activity [GO:0052689] Also known as: 2-acetyl-1-alkylglycerophosphocholine esterase activity, 1-alkyl-2-acetyl-sn-glycero-3-phosphocholine acetohydrolase activity, 1-alkyl-2-acetyl-sn-glycero-3-phosphocholine acetylhydrolase activity, LDL-PLA(2) activity, LDL-PLA2, LDL-associated phospholipase A(2) activity, LDL-associated phospholipase A2, PAF 2-acylhydrolase activity, PAF acetylhydrolase activity, alkylacetyl-GPC:acetylhydrolase activity, platelet-activating factor acetylhydrolase activity